{
  "term_id": "GO:0005634",
  "term_label": "nucleus",
  "gene_name": "Zinc finger protein 229",
  "gene": "UniProtKB:Q9UJW7",
  "gene_symbol": "ZNF229"
}